{
  "gene": "UniProtKB:P0CF75",
  "term_label": "Unknown cellular component",
  "term_id": "UNKNOWN:0003",
  "gene_name": "Endogenous Bornavirus-like nucleoprotein 1",
  "gene_symbol": "EBLN1"
}